{
  "gene": "UniProtKB:Q96H22",
  "gene_symbol": "CENPN",
  "term_label": "Unknown biological process",
  "gene_name": "Centromere protein N",
  "term_id": "UNKNOWN:0002"
}